{
  "gene": "UniProtKB:P28370",
  "gene_symbol": "SMARCA1",
  "term_id": "GO:0000785",
  "term_label": "chromatin",
  "gene_name": "Probable global transcription activator SNF2L1"
}